{
  "term_id": "GO:0035771",
  "gene": "UniProtKB:P05112",
  "term_label": "interleukin-4-mediated signaling pathway",
  "gene_name": "Interleukin-4",
  "gene_symbol": "IL4"
}